{
  "gene": "UniProtKB:Q9HBV2",
  "gene_name": "Sperm acrosome membrane-associated protein 1",
  "term_label": "acrosomal membrane",
  "term_id": "GO:0002080",
  "gene_symbol": "SPACA1"
}